{
  "gene_symbol": "DNAJC2",
  "gene": "UniProtKB:Q99543",
  "gene_name": "DnaJ homolog subfamily C member 2",
  "term_id": "GO:0030544",
  "term_label": "Hsp70 protein binding"
}